{
  "gene_symbol": "GNAI3",
  "gene_name": "Guanine nucleotide-binding protein G(i) subunit alpha-3",
  "gene": "UniProtKB:P08754",
  "term_id": "GO:0005834",
  "term_label": "heterotrimeric G-protein complex"
}